{
  "gene_symbol": "SLC35F1",
  "gene_name": "Solute carrier family 35 member F1",
  "term_label": "Unknown biological process",
  "gene": "UniProtKB:Q5T1Q4",
  "term_id": "UNKNOWN:0002"
}